{
  "term_label": "cell migration",
  "gene_name": "Cytoplasmic protein NCK2",
  "term_id": "GO:0016477",
  "gene_symbol": "NCK2",
  "gene": "UniProtKB:O43639"
}